{
  "gene": "UniProtKB:P35452",
  "gene_name": "Homeobox protein Hox-D12",
  "term_id": "UNKNOWN:0003",
  "gene_symbol": "HOXD12",
  "term_label": "Unknown cellular component"
}